inferior reticular formation development [GO:0021728] (biological process) Definition: The process whose specific outcome is the progression of the inferior reticular formation over time, from its formation to the mature structure. Sources: GOC:cls, GOC:curators, GOC:dgh, GOC:dph, GOC:jid Relationships: is_a GO:0048857; is part of medullary reticular formation development [GO:0021723]